{
  "gene": "UniProtKB:Q8TBA6",
  "gene_symbol": "GOLGA5",
  "gene_name": "Golgin subfamily A member 5",
  "term_id": "GO:0000139",
  "term_label": "Golgi membrane"
}